neurotrophin TRKA receptor binding [GO:0005168] (molecular function) Relationships: is a type of neurotrophin TRK receptor binding [GO:0005167] Also known as: neurotrophin TRKA receptor ligand Sources: GOC:ai Definition: Binding to a neurotrophin TRKA receptor.